{
  "gene": "UniProtKB:Q8N9C0",
  "gene_name": "Immunoglobulin superfamily member 22",
  "gene_symbol": "IGSF22",
  "term_id": "UNKNOWN:0001",
  "term_label": "Unknown molecular function"
}